orcinol biosynthetic process [GO:0046197] (biological process) Also known as: orcinol anabolism, orcinol biosynthesis, orcinol formation, orcinol synthesis Relationships: is a type of benzene-containing compound metabolic process [GO:0042537]; is a type of GO:0044550; is a type of GO:0046189 Sources: GOC:ai Regulation: RO_0002211 by regulation of orcinol biosynthetic process [GO:1900701]; negatively regulated by GO:1900702; positively regulated by positive regulation of orcinol biosynthetic process [GO:1900703] Definition: The chemical reactions and pathways resulting in the formation of orcinol (5-methyl-1,3-benzenediol), an aromatic compound derived from the fermentation of lichen and synthesized by some higher plants.